{
  "gene_symbol": "UHMK1",
  "gene": "UniProtKB:Q8TAS1",
  "term_id": "GO:0005634",
  "gene_name": "Serine_threonine-protein kinase Kist",
  "term_label": "nucleus"
}